positive regulation of glomerulus development [GO:0090193] (biological process) Relationships: is_a GO:0090184; is a type of regulation of glomerulus development [GO:0090192]; positively regulates glomerulus development [GO:0032835] Definition: Any process that increases the rate, frequency or extent of glomerulus development, the progression of the glomerulus over time from its initial formation until its mature state. The glomerulus is a capillary tuft surrounded by Bowman's capsule in nephrons of the vertebrate kidney. Sources: GOC:dph, GOC:tb, GOC:yaf Subtypes: positive regulation of metanephric glomerulus development [GO:0072300], positive regulation of mesonephric glomerulus development [GO:2000089]